{
  "gene_symbol": "APLP2",
  "gene_name": "Amyloid beta precursor like protein 2",
  "term_label": "axonogenesis",
  "gene": "UniProtKB:Q06481",
  "term_id": "GO:0007409"
}